{
  "gene_symbol": "RNF125",
  "gene_name": "E3 ubiquitin-protein ligase RNF125",
  "gene": "UniProtKB:Q96EQ8",
  "term_label": "ubiquitin protein ligase activity",
  "term_id": "GO:0061630"
}